{
  "gene_name": "Exosome complex component CSL4",
  "gene": "UniProtKB:Q9Y3B2",
  "term_id": "GO:0000176",
  "gene_symbol": "EXOSC1",
  "term_label": "nuclear exosome (RNase complex)"
}